{
  "gene_name": "Citron Rho-interacting kinase",
  "gene_symbol": "CIT",
  "term_label": "Unknown cellular component",
  "gene": "UniProtKB:O14578",
  "term_id": "UNKNOWN:0003"
}